{
  "gene_name": "Ankyrin repeat domain-containing protein 42",
  "term_id": "GO:0005634",
  "gene_symbol": "ANKRD42",
  "gene": "UniProtKB:Q8N9B4",
  "term_label": "nucleus"
}